{
  "term_id": "GO:0005739",
  "term_label": "mitochondrion",
  "gene": "UniProtKB:Q9NPH0",
  "gene_name": "Lysophosphatidic acid phosphatase type 6",
  "gene_symbol": "ACP6"
}